positive regulation of single-species biofilm formation [GO:1900192] (BP) Relationships: is a type of positive regulation of cellular process [GO:0048522]; is_a regulation of single-species biofilm formation [GO:1900190]; positively regulates single-species biofilm formation [GO:0044010] Also known as: up regulation of single-species biofilm formation, up-regulation of single-species biofilm formation, upregulation of single-species biofilm formation, activation of single-species biofilm formation Sources: GOC:TermGenie, GOC:di Subtypes: positive regulation of single-species biofilm formation in or on host organism [GO:1900230], GO:1900233 Definition: Any process that activates or increases the frequency, rate or extent of single-species biofilm formation.